{
  "gene": "UniProtKB:Q96B54",
  "term_label": "Unknown biological process",
  "gene_symbol": "ZNF428",
  "gene_name": "Zinc finger protein 428",
  "term_id": "UNKNOWN:0002"
}